{
  "term_label": "replication fork reversal",
  "gene_symbol": "DNA2",
  "gene": "UniProtKB:P51530",
  "term_id": "GO:0071932",
  "gene_name": "DNA replication ATP-dependent helicase_nuclease DNA2"
}